{
  "gene_symbol": "CRYGB",
  "gene": "UniProtKB:P07316",
  "term_id": "GO:0002088",
  "term_label": "lens development in camera-type eye",
  "gene_name": "Gamma-crystallin B"
}